{
  "gene_symbol": "HSPA1L",
  "term_id": "GO:0005737",
  "gene_name": "Heat shock 70 kDa protein 1-like",
  "gene": "UniProtKB:P34931",
  "term_label": "cytoplasm"
}